L-fucose metabolic process [GO:0042354] (biological process) Also known as: L-fucose metabolism Relationships: is_a fucose metabolic process [GO:0006004] Sources: GOC:jl, ISBN:0198506732 Definition: The chemical reactions and pathways involving L-fucose, 6-deoxy-L-galactose, a sugar that occurs in fucans, a class of polysaccharides in seaweeds, especially Fucus species, and in the cell wall matrix of higher plants. Subtypes: L-fucose biosynthetic process [GO:0006005], L-fucose catabolic process [GO:0042355]